{
  "gene_name": "EKC_KEOPS complex subunit TPRKB",
  "gene_symbol": "TPRKB",
  "term_label": "nucleus",
  "gene": "UniProtKB:Q9Y3C4",
  "term_id": "GO:0005634"
}